leukotriene catabolic process [GO:0036100] (biological process) Definition: The chemical reactions and pathways resulting in the breakdown of a leukotriene, a pharmacologically active substance derived from a polyunsaturated fatty acid, such as arachidonic acid. Also known as: leukotriene breakdown, leukotriene catabolism, leukotriene degradation Relationships: is a type of leukotriene metabolic process [GO:0006691]; is a type of carboxylic acid catabolic process [GO:0046395] Sources: GOC:yaf Subtypes: leukotriene B4 catabolic process [GO:0036101], leukotriene D4 catabolic process [GO:1901749], leukotriene A4 catabolic process [GO:1901752]